{
  "gene_symbol": "GCRG224",
  "gene": "UniProtKB:Q8WZA8",
  "term_label": "Unknown molecular function",
  "term_id": "UNKNOWN:0001",
  "gene_name": "Putative gastric cancer-related gene 224 protein"
}